{
  "term_id": "GO:0000796",
  "gene": "UniProtKB:Q86XI2",
  "gene_symbol": "NCAPG2",
  "term_label": "condensin complex",
  "gene_name": "Condensin-2 complex subunit G2"
}